{
  "gene": "UniProtKB:P46926",
  "gene_symbol": "GNPDA1",
  "gene_name": "Glucosamine-6-phosphate isomerase 1",
  "term_id": "GO:0006046",
  "term_label": "N-acetylglucosamine catabolic process"
}